{
  "term_id": "UNKNOWN:0001",
  "gene": "UniProtKB:Q9BRJ2",
  "gene_symbol": "MRPL45",
  "term_label": "Unknown molecular function",
  "gene_name": "Large ribosomal subunit protein mL45"
}